{
  "term_label": "cell adhesion",
  "gene_name": "Annexin A2",
  "term_id": "GO:0007155",
  "gene_symbol": "ANXA2",
  "gene": "UniProtKB:P07355"
}